{
  "term_label": "actin filament binding",
  "gene_symbol": "MYO15A",
  "term_id": "GO:0051015",
  "gene": "UniProtKB:Q9UKN7",
  "gene_name": "Unconventional myosin-XV"
}